sinapate 1-glucosyltransferase activity [GO:0050284] (molecular function) Sources: EC:2.4.1.120, MetaCyc:SINAPATE-1-GLUCOSYLTRANSFERASE-RXN Relationships: is a type of UDP-glucosyltransferase activity [GO:0035251] Definition: Catalysis of the reaction: UDP-glucose + sinapate = UDP + 1-sinapoyl-D-glucose. Also known as: UDP-glucose:sinapate D-glucosyltransferase activity, UDPglucose:sinapate D-glucosyltransferase activity, UDPglucose:sinapic acid glucosyltransferase activity, uridine 5'-diphosphoglucose-hydroxycinnamic acid acylglucosyltransferase activity, uridine diphosphoglucose-sinapate glucosyltransferase activity